{
  "term_label": "synaptic vesicle exocytosis",
  "term_id": "GO:0016079",
  "gene_name": "SNARE-associated protein Snapin",
  "gene_symbol": "SNAPIN",
  "gene": "UniProtKB:O95295"
}